{
  "gene": "UniProtKB:Q13886",
  "term_id": "GO:0005634",
  "term_label": "nucleus",
  "gene_name": "Krueppel-like factor 9",
  "gene_symbol": "KLF9"
}